inositol-3-phosphate synthase activity [GO:0004512] (molecular function) Relationships: is a type of GO:0016872 Definition: Catalysis of the reaction: D-glucose 6-phosphate = 1D-myo-inositol 3-phosphate. This reaction requires NAD, which dehydrogenates the CHOH group to CO at C-5 of the glucose 6-phosphate, making C-6 into an active methylene, able to condense with the aldehyde at C-1. Finally, the enzyme-bound NADH reconverts C-5 into the CHOH form. Sources: EC:5.5.1.4, RHEA:10716 Also known as: 1L-myo-inositol-1-phosphate lyase (isomerizing), D-glucose 6-phosphate cycloaldolase activity, glucocycloaldolase activity, glucose 6-phosphate cyclase activity, glucose-6-phosphate inositol monophosphate cycloaldolase activity, inositol 1-phosphate synthatase activity, inositol 1-phosphate synthetase activity